{
  "gene": "UniProtKB:Q9HBK9",
  "term_id": "GO:0030791",
  "gene_name": "Arsenite methyltransferase",
  "term_label": "arsenite methyltransferase activity",
  "gene_symbol": "AS3MT"
}